{
  "gene_symbol": "RABIF",
  "term_label": "guanyl-nucleotide exchange factor activity",
  "gene": "UniProtKB:P47224",
  "gene_name": "Guanine nucleotide exchange factor MSS4",
  "term_id": "GO:0005085"
}